{
  "gene_name": "E3 ubiquitin-protein ligase TRIM39",
  "gene_symbol": "TRIM39",
  "term_id": "GO:0045087",
  "term_label": "innate immune response",
  "gene": "UniProtKB:Q9HCM9"
}